{
  "gene": "UniProtKB:Q9C0A1",
  "gene_name": "Zinc finger homeobox protein 2",
  "gene_symbol": "ZFHX2",
  "term_id": "GO:0045664",
  "term_label": "regulation of neuron differentiation"
}